{
  "term_label": "nucleus",
  "term_id": "GO:0005634",
  "gene_name": "Zinc finger protein 76",
  "gene_symbol": "ZNF76",
  "gene": "UniProtKB:P36508"
}